{
  "gene_name": "Voltage-gated potassium channel subunit beta-1",
  "term_id": "GO:0008076",
  "term_label": "voltage-gated potassium channel complex",
  "gene_symbol": "KCNAB1",
  "gene": "UniProtKB:Q14722"
}